indole-3-butyrate beta-glucosyltransferase activity [GO:0052638] (molecular function) Sources: MetaCyc:RXN-11655, RHEA:62708 Relationships: is a type of UDP-glucosyltransferase activity [GO:0035251] Definition: Catalysis of the reaction: indole-3-butyrate + UDP-D-glucose = indole-3-butyryl-beta-1-D-glucose + UDP. Also known as: IBA-Glc synthetase activity, IBA-glucose synthase activity, IBAGlu synthase activity, UDP-glucose:(indol-3-yl)butyrate beta-D-glucosyltransferase activity, UDP-glucose:indol-3-ylbutyrate glucosyl-transferase activity, UDP-glucose:indol-3-ylbutyrate glucosyltransferase activity, UDPG-indol-3-ylbutyryl glucosyl transferase activity, UDPglucose:indole-3-butyrate beta-D-glucosyltransferase activity, indol-3-ylbutyrylglucose synthase activity, indole-3-butyric acid glucosyltransferase activity, uridine diphosphoglucose-indolebutyrate glucosyltransferase activity